{
  "gene": "UniProtKB:Q8NHA8",
  "term_label": "signal transduction",
  "gene_name": "Putative olfactory receptor 1F12P",
  "term_id": "GO:0007165",
  "gene_symbol": "OR1F12P"
}